host-mediated activation of viral process [GO:0044794] (biological process) Definition: A process in which a host organism initiates, promotes, or enhances the normal execution of a biological process being mediated by a virus with which it is infected. Sources: GOC:jl Also known as: positive regulation by host of viral process Relationships: is_a host-mediated perturbation of viral process [GO:0044788] Subtypes: host-mediated activation of viral transcription [GO:0043923], GO:0044829